growth factor binding [GO:0019838] (MF) Sources: GOC:curators Also known as: neurotrophin TRK receptor activity Subtypes: insulin-like growth factor binding [GO:0005520], fibroblast growth factor binding [GO:0017134], interleukin-1 binding [GO:0019966], interleukin-10 binding [GO:0019969], GO:0019970, GO:0019976, interleukin-3 binding [GO:0019978], interleukin-4 binding [GO:0019979], interleukin-5 binding [GO:0019980], interleukin-6 binding [GO:0019981], GO:0019982, interleukin-9 binding [GO:0019983], hepatocyte growth factor binding [GO:0036458], vascular endothelial growth factor binding [GO:0038085], neuregulin binding [GO:0038132], neurotrophin binding [GO:0043121], platelet-derived growth factor binding [GO:0048407], epidermal growth factor binding [GO:0048408], GO:0050431 Definition: Binding to a growth factor, proteins or polypeptides that stimulate a cell or organism to grow or proliferate. Relationships: is a type of protein binding [GO:0005515]